{
  "gene_symbol": "SELE",
  "gene_name": "E-selectin",
  "gene": "UniProtKB:P16581",
  "term_label": "response to cytokine",
  "term_id": "GO:0034097"
}